sodium-transporting ATPase activity, rotational mechanism [GO:0046962] (molecular function) Definition: Enables the transfer of a solute or solutes from one side of a membrane to the other by a rotational mechanism according to the reaction: 4 Na+(in) + ATP + H2O => 4 Na+(out) + ADP + phosphate + H+. Relationships: is a type of GO:0015081; is a type of GO:0019829; is a type of GO:0044769 Note: Found in some halophilic or alkalophilic bacteria that functions in maintaining sodium homeostasis; similar to EC:7.1.2.2 but pumps Na+ rather than H+. (Source: EC:7.2.2.1) Also known as: Na(+)-translocating ATPase activity, sodium transporting ATPase activity, rotational mechanism, Na+-translocating F1Fo-ATPase, Na+-transporting two-sector ATPase, sodium-translocating F-type ATPase activity, sodium-translocating V-type ATPase activity, sodium-transporting two-sector ATPase activity, vacuolar-type Na+-ATPase, vacuolar-type Na+-translocating ATPase, ATP phosphohydrolase (Na+-transporting) activity, ATP synthase, sodium ion specific activity, Na(+)-transporting two-sector ATPase activity, Na+-translocating ATPase activity References: PMID:30791207 Sources: RHEA:58157